stearic acid binding [GO:0070540] (molecular function) Relationships: is a type of long-chain fatty acid binding [GO:0036041] Sources: GOC:lp, GOC:mah Definition: Binding to stearic acid, the 18-carbon saturated fatty acid octadecanoic acid.